host cell surface receptor binding [GO:0046789] (molecular function) Also known as: cell surface antigen activity, host-interacting, cell surface receptor ligand References: PMID:11511370 Sources: GOC:ai Definition: Binding to a receptor on the host cell surface. Relationships: is a type of host cell surface binding [GO:0046812]; is part of adhesion of symbiont to host cell [GO:0044650]